{
  "term_id": "GO:0005737",
  "gene_symbol": "ZNG1F",
  "gene_name": "Zinc-regulated GTPase metalloprotein activator 1F",
  "gene": "UniProtKB:Q4V339",
  "term_label": "cytoplasm"
}